{
  "gene_name": "Protein ABHD8",
  "term_label": "phospholipase activity",
  "gene": "UniProtKB:Q96I13",
  "gene_symbol": "ABHD8",
  "term_id": "GO:0004620"
}